{
  "term_id": "GO:0010420",
  "gene_name": "Ubiquinone biosynthesis O-methyltransferase, mitochondrial",
  "term_label": "polyprenyldihydroxybenzoate methyltransferase activity",
  "gene_symbol": "COQ3",
  "gene": "UniProtKB:Q9NZJ6"
}